{
  "gene": "UniProtKB:Q6ZRR7",
  "gene_name": "Leucine-rich repeat-containing protein 9",
  "gene_symbol": "LRRC9",
  "term_label": "Unknown molecular function",
  "term_id": "UNKNOWN:0001"
}